vasoactive intestinal polypeptide receptor activity [GO:0004999] (MF) Sources: GOC:mah Relationships: is a type of G protein-coupled receptor activity [GO:0004930] Definition: Combining with vasoactive intestinal polypeptide to initiate a change in cell activity.